{
  "term_id": "GO:1990907",
  "gene_name": "Transcription factor 7-like 1",
  "term_label": "beta-catenin-TCF complex",
  "gene_symbol": "TCF7L1",
  "gene": "UniProtKB:Q9HCS4"
}